{
  "gene_name": "NAD-dependent protein lipoamidase sirtuin-4, mitochondrial",
  "term_label": "NAD+ poly-ADP-ribosyltransferase activity",
  "term_id": "GO:0003950",
  "gene": "UniProtKB:Q9Y6E7",
  "gene_symbol": "SIRT4"
}